{
  "term_id": "GO:0031463",
  "gene_name": "Kelch-like protein 12",
  "gene": "UniProtKB:Q53G59",
  "term_label": "Cul3-RING ubiquitin ligase complex",
  "gene_symbol": "KLHL12"
}